{
  "gene": "UniProtKB:P78537",
  "term_label": "Unknown molecular function",
  "gene_name": "Biogenesis of lysosome-related organelles complex 1 subunit 1",
  "term_id": "UNKNOWN:0001",
  "gene_symbol": "BLOC1S1"
}